{
  "gene": "UniProtKB:O43247",
  "gene_symbol": "TEX33",
  "gene_name": "Testis-expressed protein 33",
  "term_id": "UNKNOWN:0001",
  "term_label": "Unknown molecular function"
}